Barr body [GO:0001740] (cellular component) Definition: A structure found in a female mammalian cell containing an unpaired X chromosome that has become densely heterochromatic, silenced and localized at the nuclear periphery. Sources: GOC:hjd, GOC:mr, NIF_Subcellular:sao1571698684 Relationships: is a type of nuclear chromosome [GO:0000228]; is a type of X chromosome [GO:0000805]; BFO_0000051 condensed chromatin of inactivated sex chromosome [GO:0098578]